Purkinje myocyte-ventricular cardiac muscle cell adhesion involved in cell communication [GO:0086074] (biological process) Sources: GOC:BHF, GOC:mtg_cardiac_conduct_nov11 Relationships: is a type of heterotypic cell-cell adhesion [GO:0034113]; is_a GO:0086042; is part of Purkinje myocyte to ventricular cardiac muscle cell communication [GO:0086068] Definition: The attachment of an Purkinje myocyte to a ventricular cardiac muscle cell via adhesion molecules that results in the cells being juxtaposed so that they can communicate.